{
  "gene_name": "Putative protein CDKN2A-DT",
  "gene_symbol": "CDKN2A-DT",
  "gene": "UniProtKB:Q9UH64",
  "term_id": "UNKNOWN:0001",
  "term_label": "Unknown molecular function"
}